deoxycytidyl transferase activity [GO:0017125] (molecular function) Definition: Catalysis of the insertion of a dCMP residue opposite a template abasic site in DNA. References: PMID:10535901 Relationships: is a type of nucleotidyltransferase activity [GO:0016779] Also known as: deoxycytidyl transferase activity, template-dependent